{
  "gene_symbol": "USH1C",
  "term_label": "Unknown molecular function",
  "gene_name": "Harmonin",
  "gene": "UniProtKB:Q9Y6N9",
  "term_id": "UNKNOWN:0001"
}